{
  "gene": "UniProtKB:Q49MG5",
  "gene_symbol": "MAP9",
  "term_id": "GO:0090307",
  "gene_name": "Microtubule-associated protein 9",
  "term_label": "mitotic spindle assembly"
}